positive regulation of cardiac muscle tissue development [GO:0055025] (biological process) Sources: GOC:vk Definition: Any process that activates, maintains or increases the frequency, rate or extent of cardiac muscle tissue development. Relationships: is a type of positive regulation of striated muscle tissue development [GO:0045844]; is_a regulation of cardiac muscle tissue development [GO:0055024]; positively regulates GO:0048738 Also known as: positive regulation of heart muscle development, up regulation of cardiac muscle development, up-regulation of cardiac muscle development, upregulation of cardiac muscle development, activation of cardiac muscle development, stimulation of cardiac muscle development